L-ascorbic acid biosynthetic process [GO:0019853] (BP) Also known as: L-ascorbic acid anabolism, L-ascorbic acid biosynthesis, L-ascorbic acid formation, L-ascorbic acid synthesis, ascorbate biosynthesis, ascorbate biosynthetic process, vitamin C biosynthesis, vitamin C biosynthetic process Regulation: regulated by GO:2000082; negatively regulated by GO:2000083 Sources: GOC:ma, ISBN:0198547684 Subtypes: L-ascorbic acid biosynthetic process via GDP-alpha-D-mannose [GO:0090531], L-ascorbic acid biosynthetic process via UDP-alpha-D-glucuronate [GO:0090532] Definition: The chemical reactions and pathways resulting in the formation of L-ascorbic acid; L-ascorbic acid ionizes to give L-ascorbate, (2R)-2-[(1S)-1,2-dihydroxyethyl]-4-hydroxy-5-oxo-2,5-dihydrofuran-3-olate, which is required as a cofactor in the oxidation of prolyl residues to hydroxyprolyl, and other reactions. Relationships: is a type of L-ascorbic acid metabolic process [GO:0019852]; is a type of GO:0042364; is a type of GO:0046364; is a type of carboxylic acid biosynthetic process [GO:0046394]; is a type of GO:1901336